{
  "term_label": "cytoplasm",
  "gene_name": "Acyl-coenzyme A thioesterase 11",
  "term_id": "GO:0005737",
  "gene_symbol": "ACOT11",
  "gene": "UniProtKB:Q8WXI4"
}